positive regulation of retinoic acid receptor signaling pathway [GO:0048386] (biological process) Sources: GOC:dgh Definition: Any process that activates or increases the frequency, rate or extent of retinoic acid receptor signaling pathway activity. Relationships: is a type of regulation of retinoic acid receptor signaling pathway [GO:0048385]; is a type of positive regulation of intracellular signal transduction [GO:1902533]; positively regulates GO:0048384 Also known as: positive regulation of RAR signaling pathway, positive regulation of retinoic acid receptor signalling pathway, up regulation of retinoic acid receptor signaling pathway, up-regulation of retinoic acid receptor signaling pathway, upregulation of retinoic acid receptor signaling pathway, activation of retinoic acid receptor signaling pathway, stimulation of retinoic acid receptor signaling pathway